{
  "gene_name": "Aldehyde dehydrogenase family 3 member B2",
  "gene_symbol": "ALDH3B2",
  "term_label": "cytoplasm",
  "gene": "UniProtKB:P48448",
  "term_id": "GO:0005737"
}